{
  "gene_symbol": "KLHDC7A",
  "term_label": "Unknown biological process",
  "term_id": "UNKNOWN:0002",
  "gene": "UniProtKB:Q5VTJ3",
  "gene_name": "Kelch domain-containing protein 7A"
}